{
  "term_id": "GO:0004879",
  "gene_name": "Peroxisome proliferator-activated receptor gamma",
  "gene_symbol": "PPARG",
  "gene": "UniProtKB:P37231",
  "term_label": "nuclear receptor activity"
}